{
  "gene": "UniProtKB:Q5T4S7",
  "gene_symbol": "UBR4",
  "term_label": "cytoplasm protein quality control",
  "gene_name": "E3 ubiquitin-protein ligase UBR4",
  "term_id": "GO:0140455"
}